{
  "gene_name": "Non-structural maintenance of chromosomes element 3 homolog",
  "term_id": "GO:0005634",
  "term_label": "nucleus",
  "gene_symbol": "NSMCE3",
  "gene": "UniProtKB:Q96MG7"
}